deoxyguanosine catabolic process [GO:0006161] (biological process) Definition: The chemical reactions and pathways resulting in the breakdown of deoxyguanosine, a nucleoside consisting of the base guanine and the sugar deoxyribose. Also known as: deoxyguanosine breakdown, deoxyguanosine catabolism, deoxyguanosine degradation Sources: GOC:jl Relationships: is a type of purine deoxyribonucleoside catabolic process [GO:0046124]